{
  "gene_name": "Small integral membrane protein 5",
  "term_id": "UNKNOWN:0002",
  "term_label": "Unknown biological process",
  "gene": "UniProtKB:Q71RC9",
  "gene_symbol": "SMIM5"
}